{
  "term_label": "regulation of transcription by RNA polymerase II",
  "gene": "UniProtKB:A6NKF2",
  "gene_symbol": "ARID3C",
  "term_id": "GO:0006357",
  "gene_name": "AT-rich interactive domain-containing protein 3C"
}